{
  "term_id": "GO:0005789",
  "term_label": "endoplasmic reticulum membrane",
  "gene_name": "Formin-1",
  "gene_symbol": "FMN1",
  "gene": "UniProtKB:Q68DA7"
}